{
  "gene": "UniProtKB:Q86UN3",
  "gene_symbol": "RTN4RL2",
  "gene_name": "Reticulon-4 receptor-like 2",
  "term_id": "GO:0051965",
  "term_label": "positive regulation of synapse assembly"
}